{
  "term_label": "plasma membrane",
  "term_id": "GO:0005886",
  "gene_name": "Calcium homeostasis modulator protein 6",
  "gene_symbol": "CALHM6",
  "gene": "UniProtKB:Q5R3K3"
}